{
  "term_label": "pattern recognition receptor activity",
  "term_id": "GO:0038187",
  "gene_symbol": "CD209",
  "gene_name": "CD209 antigen",
  "gene": "UniProtKB:Q9NNX6"
}